{
  "gene_name": "Atrial natriuretic peptide receptor 1",
  "gene": "UniProtKB:P16066",
  "term_label": "receptor guanylyl cyclase signaling pathway",
  "gene_symbol": "NPR1",
  "term_id": "GO:0007168"
}